triose-phosphate transmembrane transporter activity [GO:0071917] (molecular function) Sources: GOC:mah, GOC:vw Definition: Enables the transfer of a triose phosphate from one side of a membrane to the other. Relationships: is a type of organophosphate ester transmembrane transporter activity [GO:0015605]; is a type of GO:1901505; is part of triose phosphate transmembrane transport [GO:0035436] Subtypes: triose-phosphate:phosphate antiporter activity [GO:0009670]